{
  "gene": "UniProtKB:Q9Y5R6",
  "term_id": "GO:0006357",
  "term_label": "regulation of transcription by RNA polymerase II",
  "gene_symbol": "DMRT1",
  "gene_name": "Doublesex- and mab-3-related transcription factor 1"
}